{
  "gene_symbol": "CSNK1A1",
  "gene_name": "Casein kinase I isoform alpha",
  "gene": "UniProtKB:P48729",
  "term_id": "GO:0007165",
  "term_label": "signal transduction"
}